{
  "gene_name": "Set1_Ash2 histone methyltransferase complex subunit ASH2",
  "gene_symbol": "ASH2L",
  "term_id": "GO:0000976",
  "gene": "UniProtKB:Q9UBL3",
  "term_label": "transcription cis-regulatory region binding"
}